{
  "term_label": "positive regulation of transcription by RNA polymerase II",
  "gene_symbol": "HOXB4",
  "term_id": "GO:0045944",
  "gene": "UniProtKB:P17483",
  "gene_name": "Homeobox protein Hox-B4"
}